{
  "term_id": "GO:0017108",
  "gene_symbol": "EXO1",
  "gene_name": "Exonuclease 1",
  "gene": "UniProtKB:Q9UQ84",
  "term_label": "5'-flap endonuclease activity"
}